{
  "term_id": "GO:0004984",
  "gene": "UniProtKB:Q8NGQ3",
  "gene_name": "Olfactory receptor 1S2",
  "gene_symbol": "OR1S2",
  "term_label": "olfactory receptor activity"
}